T=4 icosahedral viral capsid [GO:0039619] (cellular component) Relationships: is a type of icosahedral viral capsid [GO:0019030] Sources: VZ:808 Definition: The protein coat that surrounds the infective nucleic acid in some virus particles where the subunits (capsomeres) are arranged to form an icosahedron with T=4 symmetry. The T=4 capsid is composed of 12 pentameric and 30 hexameric capsomeres.